{
  "gene": "UniProtKB:O75920",
  "gene_symbol": "SERF1B",
  "term_label": "Unknown cellular component",
  "gene_name": "Small EDRK-rich factor 1",
  "term_id": "UNKNOWN:0003"
}